{
  "term_id": "UNKNOWN:0001",
  "gene": "UniProtKB:Q68CR1",
  "gene_symbol": "SEL1L3",
  "term_label": "Unknown molecular function",
  "gene_name": "Protein sel-1 homolog 3"
}